{
  "gene_symbol": "SLC10A3",
  "gene": "UniProtKB:P09131",
  "term_id": "UNKNOWN:0003",
  "gene_name": "P3 protein",
  "term_label": "Unknown cellular component"
}